multicellular organismal-level water homeostasis [GO:0050891] (biological process) Sources: GOC:dph, GOC:tb Relationships: is a type of regulation of body fluid levels [GO:0050878]; is a type of multicellular organismal-level chemical homeostasis [GO:0140962] Also known as: multicellular organismal water homeostasis, body fluid osmoregulation Subtypes: renal water homeostasis [GO:0003091] Definition: A chemical homeostatic process involved in the maintenance of a steady state level of water within extracellular body fluids, such as blood, xylem or phloem, of a multicellular organism. This is distinct from maintenance of cellular homeostasis, which occurs within a cell.